{
  "gene_symbol": "ZBED5",
  "term_id": "UNKNOWN:0002",
  "term_label": "Unknown biological process",
  "gene_name": "Zinc finger BED domain-containing protein 5",
  "gene": "UniProtKB:Q49AG3"
}